{
  "gene_symbol": "LY96",
  "term_label": "cellular response to lipopolysaccharide",
  "gene_name": "Lymphocyte antigen 96",
  "gene": "UniProtKB:Q9Y6Y9",
  "term_id": "GO:0071222"
}